{
  "gene": "UniProtKB:P59074",
  "gene_symbol": "CHMP4BP1",
  "term_label": "vesicle budding from membrane",
  "term_id": "GO:0006900",
  "gene_name": "Putative charged multivesicular body protein 4B-like protein CHMP4BP1"
}